{
  "term_id": "UNKNOWN:0001",
  "gene_symbol": "NIT1",
  "gene": "UniProtKB:Q86X76",
  "term_label": "Unknown molecular function",
  "gene_name": "Deaminated glutathione amidase"
}